heart development [GO:0007507] (biological process) Definition: The process whose specific outcome is the progression of the heart over time, from its formation to the mature structure. The heart is a hollow, muscular organ, which, by contracting rhythmically, keeps up the circulation of the blood. Relationships: is a type of animal organ development [GO:0048513]; is part of circulatory system development [GO:0072359] Sources: GOC:jid, UBERON:0000948 Subtypes: larval heart development [GO:0007508], adult heart development [GO:0007512] Also known as: dorsal vessel development, cardiac development